valine decarboxylase activity [GO:0050390] (molecular function) Relationships: is_a carboxy-lyase activity [GO:0016831] Definition: Catalysis of the reaction: L-valine + H+ = 2-methylpropanamine + CO2. Sources: EC:4.1.1.14, RHEA:18989 Also known as: L-valine carboxy-lyase (2-methylpropanamine-forming), L-valine carboxy-lyase activity, leucine decarboxylase activity